{
  "gene_symbol": "TNNC2",
  "term_label": "troponin complex",
  "gene_name": "Troponin C, skeletal muscle",
  "gene": "UniProtKB:P02585",
  "term_id": "GO:0005861"
}